{
  "term_id": "GO:0004497",
  "gene_symbol": "CYP26C1",
  "gene": "UniProtKB:Q6V0L0",
  "gene_name": "Cytochrome P450 26C1",
  "term_label": "monooxygenase activity"
}